ATPase-coupled lipo-chitin oligosaccharide transmembrane transporter activity [GO:1901514] (molecular function) Sources: GOC:TermGenie Definition: Enables the transfer of a solute or solutes from one side of a membrane to the other according to the reaction: ATP + H2O + lipo-chitin oligosaccharide(in) = ADP + phosphate + lipo-chitin oligosaccharide(out). Relationships: is a type of GO:0042626; is a type of lipo-chitin oligosaccharide transmembrane transporter activity [GO:1901513] Also known as: lipo-chitin oligosaccharide transmembrane-transporting ATPase activity